arylesterase activity [GO:0004064] (MF) Relationships: is a type of carboxylic ester hydrolase activity [GO:0052689] Also known as: A-esterase activity, paraoxonase activity, aromatic esterase, aryl-ester hydrolase Definition: Catalysis of the reaction: a phenyl acetate + H2O = a phenol + acetate. Sources: EC:3.1.1.2